{
  "gene": "UniProtKB:Q969W9",
  "gene_symbol": "PMEPA1",
  "term_label": "negative regulation of transforming growth factor beta receptor signaling pathway",
  "term_id": "GO:0030512",
  "gene_name": "Protein TMEPAI"
}